{
  "term_id": "GO:0030672",
  "term_label": "synaptic vesicle membrane",
  "gene_symbol": "SLC18A2",
  "gene_name": "Synaptic vesicular amine transporter",
  "gene": "UniProtKB:Q05940"
}